{
  "gene": "UniProtKB:Q9BZQ2",
  "gene_name": "Testicular spindle-associated protein SHCBP1L",
  "term_label": "meiotic spindle",
  "term_id": "GO:0072687",
  "gene_symbol": "SHCBP1L"
}